{
  "gene_symbol": "SPINK7",
  "term_label": "inflammatory response",
  "gene_name": "Serine protease inhibitor Kazal-type 7",
  "gene": "UniProtKB:P58062",
  "term_id": "GO:0006954"
}